pyrimidine deoxyribonucleotide interconversion [GO:0015955] (biological process) Definition: The chemical reactions and pathways by which a pyrimidine deoxyribonucleotide is synthesized from another pyrimidine deoxyribonucleotide. Sources: GOC:mah, ISBN:0306444747, ISBN:0471394831 Relationships: is a type of pyrimidine deoxyribonucleotide metabolic process [GO:0009219]; is a type of GO:0015953